{
  "term_label": "sequence-specific double-stranded DNA binding",
  "gene": "UniProtKB:Q6XYB7",
  "gene_name": "Transcription factor LBX2",
  "term_id": "GO:1990837",
  "gene_symbol": "LBX2"
}